{
  "term_id": "UNKNOWN:0001",
  "gene_name": "Ubiquitin carboxyl-terminal hydrolase 3",
  "gene_symbol": "USP3",
  "gene": "UniProtKB:Q9Y6I4",
  "term_label": "Unknown molecular function"
}